{
  "gene_symbol": "H2BC3",
  "gene_name": "Histone H2B type 1-B",
  "term_label": "extracellular space",
  "term_id": "GO:0005615",
  "gene": "UniProtKB:P33778"
}